{
  "gene": "UniProtKB:Q9UHG2",
  "term_label": "endopeptidase inhibitor activity",
  "gene_name": "ProSAAS",
  "gene_symbol": "PCSK1N",
  "term_id": "GO:0004866"
}